{
  "term_id": "GO:0004126",
  "gene": "UniProtKB:P31941",
  "gene_name": "DNA dC-dU-editing enzyme APOBEC-3A",
  "term_label": "cytidine deaminase activity",
  "gene_symbol": "APOBEC3A"
}